longitudinal side of cell surface [GO:0009930] (cellular component) Sources: GOC:mtg_sensu, GOC:sm Definition: The side of the cell parallel to the zygotic axis. Relationships: is a type of cellular anatomical structure [GO:0110165]; is part of GO:0009986